{
  "gene": "UniProtKB:Q8IX19",
  "gene_symbol": "MCEMP1",
  "term_label": "Unknown biological process",
  "gene_name": "Mast cell-expressed membrane protein 1",
  "term_id": "UNKNOWN:0002"
}